{
  "gene": "UniProtKB:Q8TBJ5",
  "gene_symbol": "FEZF2",
  "term_id": "UNKNOWN:0001",
  "term_label": "Unknown molecular function",
  "gene_name": "Fez family zinc finger protein 2"
}